negative regulation of autophagosome assembly [GO:1902902] (biological process) Relationships: is a type of GO:0016242; is a type of negative regulation of organelle assembly [GO:1902116]; is_a GO:2000785; RO_0002212 autophagosome assembly [GO:0000045] References: PMID:21975012 Sources: GOC:TermGenie, GOC:als, GOC:autophagy, GO_REF:0000058 Definition: Any process that stops, prevents or reduces the frequency, rate or extent of autophagosome assembly. Also known as: down regulation of autophagic vacuole assembly, down regulation of autophagosome biosynthesis, down regulation of autophagosome formation, down-regulation of autophagic vacuole assembly, down-regulation of autophagosome biosynthesis, down-regulation of autophagosome formation, downregulation of autophagic vacuole assembly, downregulation of autophagosome biosynthesis, downregulation of autophagosome formation, negative regulation of autophagic vacuole assembly, negative regulation of autophagosome biosynthesis, negative regulation of autophagosome formation, down regulation of PAS formation, down-regulation of PAS formation, downregulation of PAS formation, inhibition of PAS formation, inhibition of autophagic vacuole assembly, inhibition of autophagosome biosynthesis, inhibition of autophagosome formation, negative regulation of PAS formation, down regulation of autophagic vacuole formation, down-regulation of autophagic vacuole formation, downregulation of autophagic vacuole formation, inhibition of autophagic vacuole formation, negative regulation of autophagic vacuole formation